{
  "gene": "UniProtKB:Q9P2D1",
  "gene_symbol": "CHD7",
  "term_label": "chordate embryonic development",
  "term_id": "GO:0043009",
  "gene_name": "Chromodomain-helicase-DNA-binding protein 7"
}